cell cycle phase transition [GO:0044770] (biological process) Regulation: regulated by GO:1901987; RO_0002212 by negative regulation of cell cycle phase transition [GO:1901988]; RO_0002213 by positive regulation of cell cycle phase transition [GO:1901989] Also known as: cell cycle transition Sources: GOC:mtg_cell_cycle Relationships: is a type of cell cycle process [GO:0022402] Definition: The cell cycle process by which a cell commits to entering the next cell cycle phase. Subtypes: meiotic cell cycle phase transition [GO:0044771], GO:0044772, GO:0044784, cell cycle G2/M phase transition [GO:0044839], cell cycle G1/S phase transition [GO:0044843]